alpha-glucan metabolic process [GO:0030978] (biological process) Sources: GOC:mah Regulation: regulated by GO:0032948 Also known as: alpha-glucan metabolism Relationships: is a type of GO:0044042 Subtypes: GO:0030979, alpha-glucan catabolic process [GO:0030980], GO:0070595, GO:0070629 Definition: The chemical reactions and pathways involving alpha-glucans, compounds composed of glucose residues linked by alpha-D-glucosidic bonds.